{
  "gene_name": "Lysine-specific demethylase 5C",
  "term_id": "GO:0006355",
  "gene_symbol": "KDM5C",
  "term_label": "regulation of DNA-templated transcription",
  "gene": "UniProtKB:P41229"
}